{
  "term_label": "Unknown molecular function",
  "term_id": "UNKNOWN:0001",
  "gene_name": "26S proteasome non-ATPase regulatory subunit 8",
  "gene": "UniProtKB:P48556",
  "gene_symbol": "PSMD8"
}